{
  "gene_symbol": "S100A12",
  "gene_name": "Protein S100-A12",
  "term_id": "GO:0043123",
  "gene": "UniProtKB:P80511",
  "term_label": "positive regulation of canonical NF-kappaB signal transduction"
}